{
  "term_id": "GO:0005261",
  "gene_name": "Sodium leak channel NALCN",
  "gene_symbol": "NALCN",
  "gene": "UniProtKB:Q8IZF0",
  "term_label": "monoatomic cation channel activity"
}